{
  "term_label": "regulation of glucose metabolic process",
  "term_id": "GO:0010906",
  "gene_name": "[Pyruvate dehydrogenase (acetyl-transferring)] kinase isozyme 4, mitochondrial",
  "gene": "UniProtKB:Q16654",
  "gene_symbol": "PDK4"
}